{
  "term_id": "UNKNOWN:0001",
  "gene": "UniProtKB:Q5TCM9",
  "gene_name": "Late cornified envelope protein 5A",
  "gene_symbol": "LCE5A",
  "term_label": "Unknown molecular function"
}